nitroimidazole catabolic process [GO:0052804] (biological process) Definition: The chemical reactions and pathways resulting in the breakdown of nitroimidazoles, imidazole derivatives with a nitro group attached to one ring. Relationships: is a type of GO:0052805 References: PMID:16387854, PMID:19039139 Also known as: nitroimidazole breakdown, nitroimidazole catabolism, nitroimidazole degradation Subtypes: bicyclic nitroimidazole catabolic process [GO:0052800]